{
  "term_id": "UNKNOWN:0001",
  "term_label": "Unknown molecular function",
  "gene_symbol": "NPIPA9",
  "gene_name": "Nuclear pore complex-interacting protein family member A9",
  "gene": "UniProtKB:A0A0B4J1W7"
}